aldehyde dehydrogenase (NAD+) inhibitor activity [GO:0140631] (molecular function) Definition: Binds to and stops, prevents or reduces the activity of aldehyde dehydrogenase (NAD+). Relationships: is a type of enzyme inhibitor activity [GO:0004857]; negatively regulates aldehyde dehydrogenase (NAD+) activity [GO:0004029] References: PMID:33495566